{
  "gene_name": "Zinc finger protein GLIS2",
  "term_id": "GO:0045944",
  "gene": "UniProtKB:Q9BZE0",
  "gene_symbol": "GLIS2",
  "term_label": "positive regulation of transcription by RNA polymerase II"
}